{
  "term_id": "UNKNOWN:0003",
  "term_label": "Unknown cellular component",
  "gene_name": "Immunoglobulin heavy joining 2 (Fragment)",
  "gene_symbol": "IGHJ2",
  "gene": "UniProtKB:A0A0J9YWN2"
}